{
  "gene_symbol": "MX2",
  "term_id": "GO:0003924",
  "gene_name": "Interferon-induced GTP-binding protein Mx2",
  "term_label": "GTPase activity",
  "gene": "UniProtKB:P20592"
}